{
  "gene_name": "Mas-related G-protein coupled receptor member G",
  "term_id": "GO:0005886",
  "gene": "UniProtKB:Q86SM5",
  "term_label": "plasma membrane",
  "gene_symbol": "MRGPRG"
}